{
  "term_label": "Unknown molecular function",
  "term_id": "UNKNOWN:0001",
  "gene_name": "STAG3-like protein 3",
  "gene_symbol": "STAG3L3",
  "gene": "UniProtKB:P0CL85"
}